{
  "term_id": "GO:0003924",
  "term_label": "GTPase activity",
  "gene_name": "Ras-related protein Rab-2A",
  "gene_symbol": "RAB2A",
  "gene": "UniProtKB:P61019"
}